cadherin binding [GO:0045296] (MF) Relationships: is a type of cell adhesion molecule binding [GO:0050839] Subtypes: GO:0098641 Definition: Binding to cadherin, a type I membrane protein involved in cell adhesion. Sources: GOC:bf